{
  "term_label": "core mediator complex",
  "gene": "UniProtKB:Q9NVC6",
  "gene_symbol": "MED17",
  "term_id": "GO:0070847",
  "gene_name": "Mediator of RNA polymerase II transcription subunit 17"
}